{
  "gene": "UniProtKB:Q9NRX5",
  "term_label": "Unknown biological process",
  "term_id": "UNKNOWN:0002",
  "gene_symbol": "SERINC1",
  "gene_name": "Serine incorporator 1"
}